{
  "term_label": "cell-cell contact zone",
  "term_id": "GO:0044291",
  "gene": "UniProtKB:Q9BX67",
  "gene_symbol": "JAM3",
  "gene_name": "Junctional adhesion molecule C"
}